sterigmatocystin catabolic process [GO:0045574] (biological process) Sources: GOC:go_curators Relationships: is a type of toxin catabolic process [GO:0009407]; is a type of sterigmatocystin metabolic process [GO:0045460] Definition: The chemical reactions and pathways resulting in the breakdown of sterigmatocystin, a carcinogenic mycotoxin produced in high yields by strains of the common molds. Also known as: sterigmatocystin breakdown, sterigmatocystin catabolism, sterigmatocystin degradation